{
  "term_id": "GO:0005829",
  "term_label": "cytosol",
  "gene_name": "RNA-binding motif, single-stranded-interacting protein 3",
  "gene_symbol": "RBMS3",
  "gene": "UniProtKB:Q6XE24"
}